{
  "term_id": "UNKNOWN:0002",
  "term_label": "Unknown biological process",
  "gene_name": "Leucine-rich repeat-containing protein 43",
  "gene": "UniProtKB:Q8N309",
  "gene_symbol": "LRRC43"
}